{
  "term_label": "glutathione metabolic process",
  "gene": "UniProtKB:Q16775",
  "term_id": "GO:0006749",
  "gene_symbol": "HAGH",
  "gene_name": "Hydroxyacylglutathione hydrolase, mitochondrial"
}